{
  "term_label": "Unknown molecular function",
  "gene": "UniProtKB:Q9Y2I8",
  "gene_name": "WD repeat-containing protein 37",
  "term_id": "UNKNOWN:0001",
  "gene_symbol": "WDR37"
}